{
  "term_label": "integrator complex",
  "gene": "UniProtKB:Q9NVM9",
  "term_id": "GO:0032039",
  "gene_symbol": "INTS13",
  "gene_name": "Integrator complex subunit 13"
}